regulation of arginine biosynthetic process [GO:1900079] (biological process) Definition: Any process that modulates the frequency, rate or extent of arginine biosynthetic process. Relationships: is a type of GO:0062012; is a type of regulation of amino acid biosynthetic process [GO:2000282]; regulates L-arginine biosynthetic process [GO:0006526] Also known as: regulation of arginine anabolism, regulation of arginine biosynthesis, regulation of arginine formation, regulation of arginine synthesis Sources: GOC:TermGenie, GOC:dgf Subtypes: positive regulation of arginine biosynthetic process [GO:1900080], GO:2000013